{
  "gene": "UniProtKB:Q9UHC9",
  "term_label": "sterol transport",
  "gene_symbol": "NPC1L1",
  "term_id": "GO:0015918",
  "gene_name": "NPC1-like intracellular cholesterol transporter 1"
}